{
  "term_id": "GO:0000981",
  "gene": "UniProtKB:P0CG31",
  "term_label": "DNA-binding transcription factor activity, RNA polymerase II-specific",
  "gene_symbol": "ZNF286B",
  "gene_name": "Putative zinc finger protein 286B"
}